MHC class Ib protein complex binding [GO:0023025] (molecular function) Relationships: is a type of MHC protein complex binding [GO:0023023] Definition: Binding to a class Ib major histocompatibility complex. Sources: GOC:mtg_signal, GOC:vw